nor-spermidine biosynthetic process [GO:0045312] (biological process) Sources: GOC:go_curators Relationships: is a type of GO:0006596; is a type of nor-spermidine metabolic process [GO:0046204] Definition: The chemical reactions and pathways resulting in the formation of nor-spermidine, a compound related to spermidine, N-(3-aminopropyl)-1,4-diaminobutane. Also known as: nor-spermidine anabolism, nor-spermidine biosynthesis, nor-spermidine formation, nor-spermidine synthesis